{
  "gene": "UniProtKB:Q12983",
  "term_label": "nucleus",
  "gene_name": "BCL2_adenovirus E1B 19 kDa protein-interacting protein 3",
  "term_id": "GO:0005634",
  "gene_symbol": "BNIP3"
}